{
  "term_id": "UNKNOWN:0002",
  "gene_name": "Protein FAM246C",
  "gene": "UniProtKB:P0DSO1",
  "gene_symbol": "FAM246C",
  "term_label": "Unknown biological process"
}